{
  "term_label": "Unknown biological process",
  "gene_name": "Protein SSX3",
  "gene": "UniProtKB:Q99909",
  "gene_symbol": "SSX3",
  "term_id": "UNKNOWN:0002"
}